{
  "gene_symbol": "EMILIN2",
  "term_label": "Unknown molecular function",
  "gene_name": "EMILIN-2",
  "gene": "UniProtKB:Q9BXX0",
  "term_id": "UNKNOWN:0001"
}